{
  "term_id": "GO:1903278",
  "gene_symbol": "FXYD6",
  "gene": "UniProtKB:Q9H0Q3",
  "term_label": "positive regulation of sodium ion export across plasma membrane",
  "gene_name": "FXYD domain-containing ion transport regulator 6"
}